{
  "gene_name": "N-chimaerin",
  "gene_symbol": "CHN1",
  "term_id": "GO:0008045",
  "gene": "UniProtKB:P15882",
  "term_label": "motor neuron axon guidance"
}